{
  "gene_name": "Speriolin-like protein",
  "term_id": "GO:0005813",
  "term_label": "centrosome",
  "gene": "UniProtKB:Q9H0A9",
  "gene_symbol": "SPATC1L"
}